holocytochrome-c synthase activity [GO:0004408] (molecular function) Relationships: is a type of GO:0016846; is a type of GO:0140096 Definition: Catalysis of the reaction: holocytochrome c = apocytochrome c + heme. Also known as: cytochrome c heme-lyase activity, cytochrome c synthase activity, holocytochrome c synthetase activity, holocytochrome-c apocytochrome-c-lyase (heme-forming), holocytochrome-c apocytochrome-c-lyase activity Sources: EC:4.4.1.17